glutamate catabolic process to 4-hydroxybutyrate [GO:0036241] (BP) Sources: GOC:bf Note: In the catabolism of glutamate in mammals, succinate semialdehyde is converted to succinate (see GO:0006540). Plants can utilize an alternative route, converting succinic semialdehyde to 4-hydroxybutyrate using gamma-hydroxybutyrate dehydrogenase. Definition: The chemical reactions and pathways resulting in the breakdown of glutamate into 4-hydroxybutyrate. Relationships: is a type of GO:0006538; is_a short-chain fatty acid metabolic process [GO:0046459]